{
  "gene_symbol": "IGFBP6",
  "term_id": "GO:0031994",
  "gene": "UniProtKB:P24592",
  "term_label": "insulin-like growth factor I binding",
  "gene_name": "Insulin-like growth factor-binding protein 6"
}